{
  "gene": "UniProtKB:Q9P2H0",
  "term_id": "GO:0005813",
  "gene_name": "Centrosomal protein of 126 kDa",
  "gene_symbol": "CEP126",
  "term_label": "centrosome"
}